{
  "term_label": "extrinsic apoptotic signaling pathway in absence of ligand",
  "gene_symbol": "BAK1",
  "gene_name": "Bcl-2 homologous antagonist_killer",
  "gene": "UniProtKB:Q16611",
  "term_id": "GO:0097192"
}